embryonic process involved in female pregnancy [GO:0060136] (biological process) Relationships: is a type of multicellular organismal reproductive process [GO:0048609]; is part of female pregnancy [GO:0007565]; is part of embryo development ending in birth or egg hatching [GO:0009792] Sources: GOC:dph Definition: A reproductive process occurring in the embryo or fetus that allows the embryo or fetus to develop within the mother.